{
  "gene_name": "Pre-rRNA-processing protein TSR1 homolog",
  "gene_symbol": "TSR1",
  "term_id": "GO:0030686",
  "gene": "UniProtKB:Q2NL82",
  "term_label": "90S preribosome"
}